{
  "term_id": "GO:0042026",
  "gene": "UniProtKB:O60884",
  "gene_name": "DnaJ homolog subfamily A member 2",
  "term_label": "protein refolding",
  "gene_symbol": "DNAJA2"
}